midbrain development [GO:0030901] (biological process) Relationships: is a type of anatomical structure development [GO:0048856]; is part of brain development [GO:0007420] References: PMID:4975589, PMID:4992177 Definition: The process whose specific outcome is the progression of the midbrain over time, from its formation to the mature structure. The midbrain is the middle division of the three primary divisions of the developing chordate brain or the corresponding part of the adult brain (in vertebrates, includes a ventral part containing the cerebral peduncles and a dorsal tectum containing the corpora quadrigemina and that surrounds the aqueduct of Sylvius connecting the third and fourth ventricles). Also known as: mesencephalon development